{
  "term_id": "GO:0060326",
  "gene": "UniProtKB:P0DP74",
  "gene_name": "Beta-defensin 130A",
  "gene_symbol": "DEFB130A",
  "term_label": "cell chemotaxis"
}